purine deoxyribonucleotide metabolic process [GO:0009151] (biological process) Subtypes: GO:0009153, purine deoxyribonucleotide catabolic process [GO:0009155], GO:0015952, dAMP metabolic process [GO:0046053], dGMP metabolic process [GO:0046054], dADP metabolic process [GO:0046056], GO:0046060, dGDP metabolic process [GO:0046066], dGTP metabolic process [GO:0046070] Definition: The chemical reactions and pathways involving purine deoxyribonucleotide, a compound consisting of deoxyribonucleoside (a purine base linked to a deoxyribose sugar) esterified with a phosphate group at either the 3' or 5'-hydroxyl group of the sugar. Sources: GOC:go_curators, ISBN:0198506732 Relationships: is a type of purine nucleotide metabolic process [GO:0006163]; is a type of 2'-deoxyribonucleotide metabolic process [GO:0009394] Also known as: purine deoxyribonucleotide metabolism